{
  "term_label": "DNA damage checkpoint signaling",
  "gene": "UniProtKB:Q13535",
  "term_id": "GO:0000077",
  "gene_name": "Serine_threonine-protein kinase ATR",
  "gene_symbol": "ATR"
}